dolichol-linked oligosaccharide biosynthetic process [GO:0006488] (biological process) Definition: The chemical reactions and pathways resulting in the formation of dolichol-linked oligosaccharide, usually by a stepwise addition of glycosyl chains to endoplasmic reticulum membrane-bound dolichol-P. Relationships: is_a GO:1901137; is part of GO:0006487 Sources: GOC:jl, ISBN:0471331309 Also known as: N-linked glycan precursor biosynthesis, N-linked glycan precursor biosynthetic process, dolichol-linked oligosaccharide anabolism, dolichol-linked oligosaccharide biosynthesis, dolichol-linked oligosaccharide formation, dolichol-linked oligosaccharide synthesis, oligosaccharide-PP-dolichol assembly